{
  "gene": "UniProtKB:P61758",
  "term_label": "tubulin binding",
  "gene_symbol": "VBP1",
  "gene_name": "Prefoldin subunit 3",
  "term_id": "GO:0015631"
}